bronchus morphogenesis [GO:0060434] (biological process) Definition: The process in which the bronchus is generated and organized. The bronchus is the portion of the airway that connects to the lungs. Relationships: is a type of animal organ morphogenesis [GO:0009887]; is a type of tube morphogenesis [GO:0035239]; is part of bronchus development [GO:0060433] Sources: GOC:dph